{
  "gene_name": "Calcium-binding protein 4",
  "term_id": "UNKNOWN:0003",
  "gene_symbol": "CABP4",
  "gene": "UniProtKB:P57796",
  "term_label": "Unknown cellular component"
}